macromolecule transmembrane transporter activity [GO:0022884] (molecular function) Definition: Enables the transfer of a macromolecule from one side of a membrane to the other. Subtypes: protein transmembrane transporter activity [GO:0008320], polysaccharide transmembrane transporter activity [GO:0015159], lipopolysaccharide transmembrane transporter activity [GO:0015221], GO:0015438, peptidoglycan transmembrane transporter activity [GO:0015647], nucleic acid transmembrane transporter activity [GO:0051032] Sources: GOC:mtg_transport, ISBN:0815340729 Relationships: is a type of transmembrane transporter activity [GO:0022857]